{
  "gene_name": "Catenin delta-2",
  "gene_symbol": "CTNND2",
  "gene": "UniProtKB:Q9UQB3",
  "term_id": "GO:0060997",
  "term_label": "dendritic spine morphogenesis"
}